suberin biosynthetic process [GO:0010345] (BP) Relationships: is a type of phenylpropanoid biosynthetic process [GO:0009699] References: PMID:17259262 Definition: The chemical reactions and pathways resulting in the formation of suberin monomers and suberin polyesters. Suberin monomers are derived from fatty acids and trans-cinnamic acids. The monomers are then cross-linked with glycerols.